umbilical cord morphogenesis [GO:0036304] (biological process) References: PMID:15107403 Sources: GOC:BHF, GOC:gr Definition: The process in which the anatomical structures of the umbilical cord are generated and organized. The umbilical cord is an organ or embryonic origin consisting of the 2 umbilical arteries and the one umbilical vein. The umbilical cord connects the cardiovascular system of the fetus to the mother via the placenta. Relationships: is a type of anatomical structure morphogenesis [GO:0009653]; is part of umbilical cord development [GO:0061027]